{
  "term_label": "cell projection",
  "gene_name": "Spectrin beta chain, non-erythrocytic 1",
  "gene": "UniProtKB:Q01082",
  "term_id": "GO:0042995",
  "gene_symbol": "SPTBN1"
}